{
  "term_label": "muscle cell development",
  "term_id": "GO:0055001",
  "gene": "UniProtKB:P11532",
  "gene_symbol": "DMD",
  "gene_name": "Dystrophin"
}